{
  "term_label": "phosphatidylserine binding",
  "term_id": "GO:0001786",
  "gene_symbol": "ANXA1",
  "gene": "UniProtKB:P04083",
  "gene_name": "Annexin A1"
}